endoplasmic reticulum-Golgi intermediate compartment membrane [GO:0033116] (cellular component) Relationships: is a type of GO:0098588; is part of endoplasmic reticulum-Golgi intermediate compartment [GO:0005793] Also known as: ER-Golgi intermediate compartment membrane Definition: The lipid bilayer surrounding any of the compartments of the endoplasmic reticulum (ER)-Golgi intermediate compartment system. References: PMID:16723730 Sources: GOC:mah, GOC:pr